{
  "gene": "UniProtKB:Q8N668",
  "gene_name": "COMM domain-containing protein 1",
  "gene_symbol": "COMMD1",
  "term_label": "regulation of proteasomal ubiquitin-dependent protein catabolic process",
  "term_id": "GO:0032434"
}